{
  "gene_symbol": "RUNX3",
  "gene_name": "Runt-related transcription factor 3",
  "term_label": "neuron differentiation",
  "gene": "UniProtKB:Q13761",
  "term_id": "GO:0030182"
}